flavonol binding [GO:0097244] (MF) Relationships: is a type of GO:0043168; is a type of flavonoid binding [GO:0097243] Definition: Binding to a flavonol, a flavonoid that contains a 3-hydroxy-2-phenylchromen-4-one backbone. Sources: GOC:sl